{
  "gene_name": "Protein N-terminal glutamine amidohydrolase",
  "gene": "UniProtKB:Q96HA8",
  "term_label": "Unknown biological process",
  "term_id": "UNKNOWN:0002",
  "gene_symbol": "NTAQ1"
}